{
  "gene_name": "Iodotyrosine deiodinase 1",
  "term_id": "GO:0042403",
  "gene": "UniProtKB:Q6PHW0",
  "term_label": "thyroid hormone metabolic process",
  "gene_symbol": "IYD"
}